collagen receptor activity [GO:0038064] (MF) Definition: Combining with a collagen and transmitting the signal from one side of the membrane to the other to initiate a change in cell activity. Also known as: transmembrane collagen receptor activity References: PMID:21568710 Sources: GOC:bf, GOC:uh Subtypes: protein tyrosine kinase collagen receptor activity [GO:0038062] Relationships: is a type of transmembrane signaling receptor activity [GO:0004888]; is part of collagen-activated signaling pathway [GO:0038065]; has part collagen binding [GO:0005518]